positive regulation of myeloid dendritic cell cytokine production [GO:0002735] (biological process) Definition: Any process that activates or increases the frequency, rate, or extent of myeloid dendritic cell cytokine production. Also known as: up regulation of myeloid dendritic cell cytokine production, up-regulation of myeloid dendritic cell cytokine production, upregulation of myeloid dendritic cell cytokine production, activation of myeloid dendritic cell cytokine production, stimulation of myeloid dendritic cell cytokine production Sources: GOC:add Relationships: is a type of GO:0002732; is a type of regulation of myeloid dendritic cell cytokine production [GO:0002733]; is a type of positive regulation of myeloid leukocyte mediated immunity [GO:0002888]; is_a positive regulation of myeloid leukocyte cytokine production involved in immune response [GO:0061081]; positively regulates myeloid dendritic cell cytokine production [GO:0002372]